{
  "term_id": "UNKNOWN:0003",
  "gene": "UniProtKB:A6NHG9",
  "gene_symbol": "OR5H14",
  "gene_name": "Olfactory receptor 5H14",
  "term_label": "Unknown cellular component"
}